protein C inhibitor-TMPRSS7 complex [GO:0036024] (cellular component) Relationships: is a type of serine protease inhibitor complex [GO:0097180] Definition: A heterodimeric protein complex that contains protein C inhibitor (SERPINA5) and transmembrane protease serine 7 (TMPRSS7); formation of the complex inhibits the serine protease activity of transmembrane protease serine 7. Also known as: PCI-TMPRSS7 complex, SERPINA5-TMPRSS7 complex, plasma serine protease inhibitor-TMPRSS7 complex, protein C inhibitor-matriptase-3 complex, protein C inhibitor-transmembrane protease serine 7 complex, serpin A5-TMPRSS7 complex References: PMID:15853774 Sources: GOC:ans